{
  "gene_symbol": "MOG",
  "gene": "UniProtKB:Q16653",
  "term_id": "GO:0009897",
  "gene_name": "Myelin-oligodendrocyte glycoprotein",
  "term_label": "external side of plasma membrane"
}